Golgi organization [GO:0007030] (biological process) Sources: GOC:dph, GOC:jl, GOC:mah Subtypes: GO:0048280, Golgi inheritance [GO:0048313], Golgi ribbon formation [GO:0090161], Golgi disassembly [GO:0090166], Golgi distribution to daughter cells [GO:0090167], GO:0090168 Relationships: is a type of organelle organization [GO:0006996]; BFO_0000050 endomembrane system organization [GO:0010256] Definition: A process that is carried out at the cellular level which results in the assembly, arrangement of constituent parts, or disassembly of the Golgi apparatus. Also known as: Golgi apparatus organization, Golgi organisation, Golgi organization and biogenesis Regulation: regulated by regulation of Golgi organization [GO:1903358]